{
  "gene": "UniProtKB:Q8IYM0",
  "term_id": "UNKNOWN:0001",
  "term_label": "Unknown molecular function",
  "gene_name": "Protein FAM186B",
  "gene_symbol": "FAM186B"
}